nuclear glucocorticoid receptor activity [GO:0004883] (molecular function) Subtypes: nuclear cortisol receptor activity [GO:0031963] Definition: A nuclear receptor activity regulated by glucocorticoid binding and modulating the transcription of specific gene sets transcribed by RNA polymerase II. Also known as: glucocorticoid receptor activity Relationships: is a type of GO:0003707; is part of nuclear receptor-mediated glucocorticoid signaling pathway [GO:0042921] References: PMID:17689856, PMID:20920967 Sources: GOC:signaling